{
  "term_label": "cobalamin binding",
  "gene": "UniProtKB:P20061",
  "gene_symbol": "TCN1",
  "gene_name": "Transcobalamin-1",
  "term_id": "GO:0031419"
}